{
  "gene_symbol": "NMU",
  "gene_name": "Neuromedin-U",
  "term_id": "GO:0007218",
  "term_label": "neuropeptide signaling pathway",
  "gene": "UniProtKB:P48645"
}